positive regulation of melanocyte differentiation [GO:0045636] (biological process) Subtypes: positive regulation of early stripe melanocyte differentiation [GO:0050948], positive regulation of late stripe melanocyte differentiation [GO:0050950] Also known as: positive regulation of melanophore differentiation, up regulation of melanocyte differentiation, up-regulation of melanocyte differentiation, upregulation of melanocyte differentiation, activation of melanocyte differentiation, stimulation of melanocyte differentiation Definition: Any process that activates or increases the frequency, rate or extent of melanocyte differentiation. Relationships: is a type of regulation of melanocyte differentiation [GO:0045634]; is a type of positive regulation of pigment cell differentiation [GO:0050942]; RO_0002213 melanocyte differentiation [GO:0030318] Sources: GOC:go_curators